(R)-3-hydroxyacid-ester dehydrogenase activity [GO:0047108] (molecular function) Relationships: is a type of GO:0016616 Definition: Catalysis of the reaction: ethyl (R)-3-hydroxyhexanoate + NADP+ = ethyl 3-oxohexanoate + H+ + NADPH. Sources: EC:1.1.1.279, RHEA:24352 Also known as: (R)-3-hydroxyacid ester dehydrogenase activity, 3-oxo ester (R)-reductase activity, ethyl-(R)-3-hydroxyhexanoate:NADP+ 3-oxidoreductase activity